molybdenum ion binding [GO:0030151] (molecular function) Also known as: Mo ion binding, molybdenum binding Relationships: is a type of transition metal ion binding [GO:0046914] Sources: GOC:ai Definition: Binding to a molybdenum ion (Mo).